{
  "gene_name": "Fractalkine",
  "term_label": "eosinophil chemotaxis",
  "term_id": "GO:0048245",
  "gene": "UniProtKB:P78423",
  "gene_symbol": "CX3CL1"
}